{
  "gene_symbol": "PERP",
  "term_label": "cell-cell junction",
  "gene_name": "p53 apoptosis effector related to PMP-22",
  "gene": "UniProtKB:Q96FX8",
  "term_id": "GO:0005911"
}